{
  "gene_symbol": "CAVIN4",
  "gene": "UniProtKB:Q5BKX8",
  "term_label": "caveola",
  "term_id": "GO:0005901",
  "gene_name": "Caveolae-associated protein 4"
}